intestinal epithelial cell maturation [GO:0060574] (biological process) References: PMID:18824147 Sources: GOC:dph Definition: The developmental process, independent of morphogenetic (shape) change, that is required for a columna/cuboidal epithelial cell of the intestine to attain its fully functional state. A columnar/cuboidal epithelial cell of the intestine mature as they migrate from the intestinal crypt to the villus. Relationships: is a type of columnar/cuboidal epithelial cell maturation [GO:0002069]; is part of intestinal epithelial cell development [GO:0060576]